{
  "gene": "UniProtKB:O60238",
  "gene_symbol": "BNIP3L",
  "term_id": "GO:0097345",
  "gene_name": "BCL2_adenovirus E1B 19 kDa protein-interacting protein 3-like",
  "term_label": "mitochondrial outer membrane permeabilization"
}